{
  "gene_symbol": "PCNX3",
  "gene": "UniProtKB:Q9H6A9",
  "term_label": "Unknown cellular component",
  "term_id": "UNKNOWN:0003",
  "gene_name": "Pecanex-like protein 3"
}